histone H3 reader activity [GO:0140006] (molecular function) Relationships: is a type of histone reader activity [GO:0140566] Subtypes: histone H3K27me3 reader activity [GO:0061628], histone H3K9me2/3 reader activity [GO:0062072], histone H3K4me3 reader activity [GO:0140002], GO:0140003, histone H3Q5ser reader activity [GO:0140004], histone H3K14ac reader activity [GO:0140015], histone H3K18cr reader activity [GO:0140017], GO:0140019, GO:0140038, histone H3K18ac reader activity [GO:0140044], GO:0140072, histone H3K4me1 reader activity [GO:0140109], histone H3K23ac reader activity [GO:0140118], histone H3K27ac reader activity [GO:0140119], histone H3R8me2 reader activity [GO:0140127], histone H3K56ac reader activity [GO:0140129], histone H3K18ub reader activity [GO:0140254], histone H3K23ub reader activity [GO:0140257], histone H3K14ub reader activity [GO:0140258] Definition: A histone reader that specifically binds either to an unmodified histone H3 or a form modified by a post-translational modification on a specific residue. The most common PTMs on histones are methylation, acetylation and phosphorylation. References: PMID:11498575, PMID:25688442, PMID:31082667, PMID:34726351